{
  "gene_name": "Protein FAM90A17",
  "term_label": "Unknown biological process",
  "gene": "UniProtKB:P0DV74",
  "term_id": "UNKNOWN:0002",
  "gene_symbol": "FAM90A17"
}